regulation of dopamine secretion [GO:0014059] (biological process) Sources: GOC:ef Definition: Any process that modulates the frequency, rate or extent of the regulated release of dopamine. Relationships: is a type of regulation of catecholamine secretion [GO:0050433]; regulates dopamine secretion [GO:0014046] Subtypes: negative regulation of dopamine secretion [GO:0033602], GO:0033603